phosphatidylinositol-4-phosphate-cholesterol exchange activity [GO:0160291] (molecular function) Definition: Catalysis of the reaction: a 1,2-diacyl-sn-glycero-3-phospho-(1D-myo-inositol 4-phosphate)(out) + cholesterol(in) = 1,2-diacyl-sn-glycero-3-phospho-(1D-myo-inositol 4-phosphate)(in) + cholesterol(out). This reaction results in the exchange of cholesterol for phosphatidylinositol-4-phosphate (PI(4)P) between membranes. References: PMID:24209621, PMID:29596003 Relationships: is_a GO:0008526; is a type of cholesterol transfer activity [GO:0120020]; is a type of lipid exchange activity [GO:7770011]